{
  "gene_symbol": "GDPD1",
  "gene_name": "Lysophospholipase D GDPD1",
  "gene": "UniProtKB:Q8N9F7",
  "term_id": "GO:0046475",
  "term_label": "glycerophospholipid catabolic process"
}